{
  "gene_name": "Melanoma-associated antigen 6",
  "term_label": "negative regulation of transcription by RNA polymerase II",
  "term_id": "GO:0000122",
  "gene_symbol": "MAGEA6",
  "gene": "UniProtKB:P43360"
}